{
  "term_label": "heterochromatin formation",
  "gene_symbol": "H2AL3",
  "term_id": "GO:0031507",
  "gene_name": "Histone H2A-like 3",
  "gene": "UniProtKB:A0A3B3IU63"
}